XTP diphosphatase activity [GO:0036222] (MF) Note: While XTP is not produced by cells, deamination of purine bases can result in accumulation of such nucleotides as ITP, dITP, XTP, and dXTP. XTPase contributes to the removal of these abnormal bases from the cellular pool of nucleotide triphosphates. Definition: Catalysis of the reaction: XTP + H2O = XMP + H+ + diphosphate. References: PMID:16216582, PMID:22531138 Sources: GOC:pz, RHEA:28610 Relationships: is a type of nucleoside triphosphate diphosphatase activity [GO:0047429] Also known as: XTP pyrophosphohydrolase activity, XTPase activity, XTP/dITP diphosphatase, hypoxanthine/xanthine dNTP pyrophosphatase